{
  "term_label": "mitochondrial electron transport, cytochrome c to oxygen",
  "gene": "UniProtKB:P13073",
  "term_id": "GO:0006123",
  "gene_symbol": "COX4I1",
  "gene_name": "Cytochrome c oxidase subunit 4 isoform 1, mitochondrial"
}